{
  "gene_name": "Melanocyte-stimulating hormone receptor",
  "gene_symbol": "MC1R",
  "term_label": "melanocyte-stimulating hormone receptor activity",
  "gene": "UniProtKB:Q01726",
  "term_id": "GO:0004980"
}